growth plate cartilage development [GO:0003417] (biological process) Sources: GOC:ascb_2009, GOC:dph, GOC:tb Definition: The process whose specific outcome is the progression of the cartilage that will provide a scaffold for mineralization of endochondral bones as they elongate or grow. Relationships: is a type of GO:0060351; is a type of GO:0061448; is part of endochondral bone growth [GO:0003416]